{
  "term_id": "UNKNOWN:0001",
  "gene_symbol": "LTF",
  "term_label": "Unknown molecular function",
  "gene": "UniProtKB:P02788",
  "gene_name": "Lactotransferrin"
}